{
  "gene_name": "Tetraspanin-10",
  "term_id": "GO:0005886",
  "term_label": "plasma membrane",
  "gene": "UniProtKB:Q9H1Z9",
  "gene_symbol": "TSPAN10"
}